{
  "term_id": "GO:0006302",
  "gene_symbol": "RAD50",
  "gene": "UniProtKB:Q92878",
  "term_label": "double-strand break repair",
  "gene_name": "DNA repair protein RAD50"
}